{
  "term_label": "Unknown molecular function",
  "gene_symbol": "RPN2",
  "gene_name": "Dolichyl-diphosphooligosaccharide--protein glycosyltransferase subunit 2",
  "term_id": "UNKNOWN:0001",
  "gene": "UniProtKB:P04844"
}